{
  "gene_symbol": "NDUFV1-DT",
  "gene_name": "Uncharacterized protein NDUFV1-DT",
  "gene": "UniProtKB:Q8NBR9",
  "term_label": "Unknown molecular function",
  "term_id": "UNKNOWN:0001"
}